{
  "gene_symbol": "VPS35",
  "gene_name": "Vacuolar protein sorting-associated protein 35",
  "term_label": "retromer complex",
  "term_id": "GO:0030904",
  "gene": "UniProtKB:Q96QK1"
}